{
  "term_id": "GO:1990756",
  "gene_symbol": "PRAMEF10",
  "gene_name": "PRAME family member 10",
  "gene": "UniProtKB:O60809",
  "term_label": "ubiquitin-like ligase-substrate adaptor activity"
}